meiotic telomere clustering [GO:0045141] (biological process) Subtypes: GO:0044821 Definition: The cell cycle process in which the dynamic reorganization of telomeres occurs in early meiotic prophase, during which meiotic chromosome ends are gathered in a bouquet arrangement at the inner surface of the nuclear envelope proximal to the spindle pole body. This plays an important role in progression through meiosis and precedes synapsis. References: PMID:10690419 Sources: GOC:vw Also known as: bouquet biosynthesis, bouquet formation Relationships: is a type of telomere localization [GO:0034397]; is a type of chromosome organization involved in meiotic cell cycle [GO:0070192]; is a type of chromosome localization to nuclear envelope involved in homologous chromosome segregation [GO:0090220]